{
  "gene": "UniProtKB:P05451",
  "term_id": "GO:0005179",
  "gene_name": "Lithostathine-1-alpha",
  "term_label": "hormone activity",
  "gene_symbol": "REG1A"
}